N-acetylneuraminate 9-O-acetyltransferase activity [GO:0047186] (molecular function) Also known as: sialate O-acetyltransferase, N-acetylneuraminate 7-O(or 9-O)-acetyltransferase activity, N-acetylneuraminate 7(8)-O-acetyltransferase activity, N-acetylneuraminate 7,8-O-acetyltransferase activity, N-acetylneuraminate O7-(or O9-)acetyltransferase activity, acetyl-CoA:N-acetylneuraminate 7-O(or 9-O)-acetyltransferase activity, acetyl-CoA:N-acetylneuraminate-7- and/or 8-O-acetyltransferase activity, acetyl-CoA:N-acetylneuraminate-7- or 8-O-acetyltransferase activity, acetyl-CoA:N-acetylneuraminate-9(7)-O-acetyltransferase activity, acetyl-CoA:N-acetylneuraminate-9(or 7)-O-acetyltransferase activity, glycoprotein 7(9)-O-acetyltransferase activity Definition: Catalysis of the reaction: CMP-N-acetyl-beta-neuraminate + acetyl-CoA = CMP-N-acetyl-9-O-acetyl-beta-neuraminate + CoA. Relationships: is a type of O-acetyltransferase activity [GO:0016413] Sources: EC:2.3.1.45, RHEA:81827